{
  "gene_name": "Alpha-1,3-mannosyl-glycoprotein 4-beta-N-acetylglucosaminyltransferase B",
  "gene_symbol": "MGAT4B",
  "term_id": "GO:0008375",
  "term_label": "acetylglucosaminyltransferase activity",
  "gene": "UniProtKB:Q9UQ53"
}